{
  "term_label": "RNA polymerase binding",
  "term_id": "GO:0070063",
  "gene_name": "Transcription elongation regulator 1-like protein",
  "gene": "UniProtKB:Q5VWI1",
  "gene_symbol": "TCERG1L"
}